4-vinylanisole biosynthetic process [GO:0160305] (biological process) References: PMID:40562929 Definition: The chemical reactions and pathways resulting in the formation of 4-vinylanisole. 4-vinylanisole derived from food plant phenylalanin is the aggregation pheromone specifically released by gregarious migratory locusts. Relationships: is a type of pheromone biosynthetic process [GO:0042811]